{
  "term_id": "GO:0030594",
  "gene_name": "5-hydroxytryptamine receptor 1D",
  "gene_symbol": "HTR1D",
  "term_label": "neurotransmitter receptor activity",
  "gene": "UniProtKB:P28221"
}